{
  "term_label": "positive regulation of anaphase-promoting complex-dependent catabolic process",
  "gene_name": "Cell division cycle protein 20 homolog B",
  "term_id": "GO:1905786",
  "gene_symbol": "CDC20B",
  "gene": "UniProtKB:Q86Y33"
}